{
  "gene": "UniProtKB:Q5VST9",
  "gene_symbol": "OBSCN",
  "term_id": "GO:0042383",
  "term_label": "sarcolemma",
  "gene_name": "Obscurin"
}